{
  "term_id": "GO:0006357",
  "gene_name": "Zinc finger homeobox protein 4",
  "gene": "UniProtKB:Q86UP3",
  "term_label": "regulation of transcription by RNA polymerase II",
  "gene_symbol": "ZFHX4"
}